{
  "gene": "UniProtKB:Q12931",
  "gene_symbol": "TRAP1",
  "term_label": "ATP hydrolysis activity",
  "gene_name": "Heat shock protein 75 kDa, mitochondrial",
  "term_id": "GO:0016887"
}